{
  "term_label": "signal transduction",
  "gene_symbol": "RHOBTB2",
  "gene": "UniProtKB:Q9BYZ6",
  "gene_name": "Rho-related BTB domain-containing protein 2",
  "term_id": "GO:0007165"
}